{
  "gene_symbol": "CSNK2A3",
  "term_id": "GO:0004674",
  "gene": "UniProtKB:Q8NEV1",
  "term_label": "protein serine/threonine kinase activity",
  "gene_name": "Casein kinase II subunit alpha 3"
}